{
  "term_label": "NAADP-sensitive calcium-release channel activity",
  "gene_symbol": "MCOLN3",
  "gene": "UniProtKB:Q8TDD5",
  "term_id": "GO:0072345",
  "gene_name": "Mucolipin-3"
}